regulation of emericellamide biosynthetic process [GO:1900658] (biological process) Subtypes: negative regulation of emericellamide biosynthetic process [GO:1900659], GO:1900660, regulation of emericellamide A biosynthetic process [GO:1900661] Sources: GOC:TermGenie, GOC:di Definition: Any process that modulates the frequency, rate or extent of emericellamide biosynthetic process. Also known as: regulation of emericellamide anabolism, regulation of emericellamide biosynthesis, regulation of emericellamide formation, regulation of emericellamide synthesis Relationships: is a type of regulation of amide metabolic process [GO:0034248]; is a type of regulation of lipid biosynthetic process [GO:0046890]; is a type of regulation of small molecule metabolic process [GO:0062012]; is a type of regulation of secondary metabolite biosynthetic process [GO:1900376]; regulates emericellamide biosynthetic process [GO:1900557]